{
  "term_label": "Unknown molecular function",
  "gene": "UniProtKB:Q9NRR3",
  "term_id": "UNKNOWN:0001",
  "gene_name": "CDC42 small effector protein 2",
  "gene_symbol": "CDC42SE2"
}